outward rectifier potassium channel inhibitor activity [GO:0140628] (molecular function) Definition: Binds to and stops, prevents, or reduces the activity of an outwardly rectifying potassium channel. References: PMID:28108814 Relationships: is_a potassium channel inhibitor activity [GO:0019870]; negatively regulates outward rectifier potassium channel activity [GO:0015271]